{
  "gene": "UniProtKB:Q9NP97",
  "gene_symbol": "DYNLRB1",
  "term_label": "dynein intermediate chain binding",
  "gene_name": "Dynein light chain roadblock-type 1",
  "term_id": "GO:0045505"
}